anterior lateral line neuromast development [GO:0048901] (biological process) Sources: ISBN:0125296509 Relationships: is a type of neuromast development [GO:0048884]; is part of anterior lateral line development [GO:0048899] Definition: The process whose specific outcome is the progression of the anterior lateral line neuromast over time, from its formation to the mature structure. The neuromast is the sensory receptor of the anterior lateral line system and is composed of a population of sensory hair cells, and nonsensory supporting cells and mantle cells. Neuromast are located superficially on the epithelium or in lateral line canals.